chloramphenicol O-acetyltransferase activity [GO:0008811] (MF) Also known as: CAT I, CAT II, CAT III, acetyl-CoA:chloramphenicol 3-O-acetyltransferase activity, chloramphenicol acetylase activity, chloramphenicol acetyltransferase activity, chloramphenicol transacetylase activity Definition: Catalysis of the reaction: chloramphenicol + acetyl-CoA = chloramphenicol 3-acetate + CoA. Sources: EC:2.3.1.28, RHEA:18421 Relationships: is a type of O-acetyltransferase activity [GO:0016413]